{
  "gene_name": "Vacuolar protein sorting-associated protein 8 homolog",
  "gene_symbol": "VPS8",
  "term_label": "endosomal vesicle fusion",
  "term_id": "GO:0034058",
  "gene": "UniProtKB:Q8N3P4"
}